smooth septate junction assembly [GO:0090528] (biological process) Definition: The assembly of a smooth septate junction, a septate junction that lacks the regular arrays of electron-dense septae found in pleated septate junctions. Relationships: is a type of septate junction assembly [GO:0019991] References: PMID:22854041